{
  "gene_name": "Sterile alpha motif domain-containing protein 14",
  "gene": "UniProtKB:Q8IZD0",
  "gene_symbol": "SAMD14",
  "term_id": "GO:0007015",
  "term_label": "actin filament organization"
}